thiamine transport [GO:0015888] (biological process) Subtypes: thiamine transmembrane transport [GO:0071934] Relationships: is a type of GO:0015695; is a type of vitamin transport [GO:0051180]; is a type of nitrogen compound transport [GO:0071705]; is a type of GO:0072348 Sources: GOC:ai Definition: The directed movement of thiamine into, out of or within a cell, or between cells, by means of some agent such as a transporter or pore. Thiamine is vitamin B1, a water soluble vitamin present in fresh vegetables and meats, especially liver. Also known as: thiamin transport, vitamin B1 transport